{
  "gene_name": "E3 ubiquitin-protein ligase HECW1",
  "term_id": "GO:0061630",
  "gene": "UniProtKB:Q76N89",
  "term_label": "ubiquitin protein ligase activity",
  "gene_symbol": "HECW1"
}